{
  "gene_symbol": "EXOSC1",
  "term_label": "Unknown molecular function",
  "term_id": "UNKNOWN:0001",
  "gene_name": "Exosome complex component CSL4",
  "gene": "UniProtKB:Q9Y3B2"
}